regulation of protein localization to spindle pole body [GO:1902363] (biological process) Also known as: regulation of protein localisation to spindle pole body Subtypes: regulation of protein localization to meiotic spindle pole body [GO:0140433], negative regulation of protein localization to spindle pole body [GO:1902364], positive regulation of protein localization to spindle pole body [GO:1902365], regulation of protein localization to mitotic spindle pole body [GO:1902542] Relationships: is a type of regulation of protein localization [GO:0032880]; regulates protein localization to spindle pole body [GO:0071988] Definition: Any process that modulates the frequency, rate or extent of protein localization to spindle pole body. References: PMID:21131906 Sources: GOC:TermGenie